{
  "gene_name": "Epithelial membrane protein 3",
  "term_label": "Unknown molecular function",
  "gene_symbol": "EMP3",
  "term_id": "UNKNOWN:0001",
  "gene": "UniProtKB:P54852"
}